{
  "term_id": "UNKNOWN:0002",
  "gene_name": "Prolyl endopeptidase",
  "gene_symbol": "PREP",
  "gene": "UniProtKB:P48147",
  "term_label": "Unknown biological process"
}